{
  "term_id": "GO:0006887",
  "gene_symbol": "CDK16",
  "term_label": "exocytosis",
  "gene": "UniProtKB:Q00536",
  "gene_name": "Cyclin-dependent kinase 16"
}